{
  "gene": "UniProtKB:P20309",
  "gene_symbol": "CHRM3",
  "term_label": "G protein-coupled acetylcholine receptor activity",
  "gene_name": "Muscarinic acetylcholine receptor M3",
  "term_id": "GO:0016907"
}